{
  "gene_symbol": "UBXN8",
  "term_id": "UNKNOWN:0002",
  "gene": "UniProtKB:O00124",
  "gene_name": "UBX domain-containing protein 8",
  "term_label": "Unknown biological process"
}